{
  "gene": "UniProtKB:A6NJG6",
  "term_label": "regulation of transcription by RNA polymerase II",
  "term_id": "GO:0006357",
  "gene_name": "Arginine-fifty homeobox",
  "gene_symbol": "ARGFX"
}